{
  "term_id": "GO:0005737",
  "gene": "UniProtKB:P13928",
  "gene_name": "Annexin A8",
  "gene_symbol": "ANXA8",
  "term_label": "cytoplasm"
}